deoxyadenosine metabolic process [GO:0046090] (biological process) Subtypes: deoxyadenosine catabolic process [GO:0006157], GO:0046091 Relationships: is a type of purine deoxyribonucleoside metabolic process [GO:0046122] Definition: The chemical reactions and pathways involving deoxyadenosine, 2-deoxyribosyladenine, one of the four major nucleosides of DNA. Sources: GOC:go_curators Also known as: deoxyadenosine metabolism